{
  "term_label": "microtubule motor activity",
  "term_id": "GO:0003777",
  "gene_name": "Kinesin-like protein KIF21A",
  "gene_symbol": "KIF21A",
  "gene": "UniProtKB:Q7Z4S6"
}